acetylglucosaminyltransferase activity [GO:0008375] (molecular function) Relationships: is_a UDP-glycosyltransferase activity [GO:0008194]; is a type of hexosyltransferase activity [GO:0016758] Sources: ISBN:0198506732 Definition: Catalysis of the transfer of an N-acetylglucosaminyl residue from UDP-N-acetyl-glucosamine to a sugar. Subtypes: glucuronyl-galactosyl-proteoglycan 4-alpha-N-acetylglucosaminyltransferase activity [GO:0001888], alpha-1,3-mannosylglycoprotein 2-beta-N-acetylglucosaminyltransferase activity [GO:0003827], GO:0003829, GO:0003830, GO:0004100, dolichyl-phosphate alpha-N-acetylglucosaminyltransferase activity [GO:0004166], N-acetylglucosaminyldiphosphodolichol N-acetylglucosaminyltransferase activity [GO:0004577], N-acetyllactosaminide beta-1,6-N-acetylglucosaminyltransferase activity [GO:0008109], alpha-1,3-mannosylglycoprotein 4-beta-N-acetylglucosaminyltransferase activity [GO:0008454], alpha-1,6-mannosylglycoprotein 2-beta-N-acetylglucosaminyltransferase activity [GO:0008455], GO:0008532, lipopolysaccharide N-acetylglucosaminyltransferase activity [GO:0008917], GO:0016262, phosphatidylinositol N-acetylglucosaminyltransferase activity [GO:0017176], alpha-1,6-mannosylglycoprotein 6-beta-N-acetylglucosaminyltransferase activity [GO:0030144], high-mannose-oligosaccharide beta-1,4-N-acetylglucosaminyltransferase activity [GO:0033827], O-fucosylpeptide 3-beta-N-acetylglucosaminyltransferase activity [GO:0033829], Skp1-protein-hydroxyproline N-acetylglucosaminyltransferase activity [GO:0033830], heparan sulfate N-acetylglucosaminyltransferase activity [GO:0042328], beta-1,4-mannosylglycolipid beta-1,3-N-acetylglucosaminyltransferase activity [GO:0046981], GO:0047222, GO:0047223, GO:0047224, acetylgalactosaminyl-O-glycosyl-glycoprotein beta-1,6-N-acetylglucosaminyltransferase activity [GO:0047225], alpha-1,6-mannosylglycoprotein 4-beta-N-acetylglucosaminyltransferase activity [GO:0047253], lactosylceramide 1,3-N-acetyl-beta-D-glucosaminyltransferase activity [GO:0047256], steroid N-acetylglucosaminyltransferase activity [GO:0047261], poly(ribitol-phosphate) N-acetylglucosaminyltransferase activity [GO:0047269], GO:0050508, undecaprenyldiphospho-muramoylpentapeptide beta-N-acetylglucosaminyltransferase activity [GO:0050511], UDP-N-acetyl-D-glucosamine:N-acetylmuramoyl-L-alanyl-D-glutamyl-meso-2,6-diaminopimelyl-D-alanyl-D-alanine-diphosphoundecaprenol 4-beta-N-acetylglucosaminlytransferase activity [GO:0051991], protein O-acetylglucosaminyltransferase activity [GO:0097363] Also known as: GlcNAc transferase activity